{
  "term_id": "GO:0006511",
  "gene_name": "E3 ubiquitin-protein ligase RNF213",
  "gene": "UniProtKB:Q63HN8",
  "gene_symbol": "RNF213",
  "term_label": "ubiquitin-dependent protein catabolic process"
}